{
  "gene_name": "Nuclear protein localization protein 4 homolog",
  "gene": "UniProtKB:Q8TAT6",
  "gene_symbol": "NPLOC4",
  "term_id": "GO:0031625",
  "term_label": "ubiquitin protein ligase binding"
}